{
  "term_label": "negative regulation of hippo signaling",
  "gene_name": "Striatin-interacting protein 2",
  "gene_symbol": "STRIP2",
  "gene": "UniProtKB:Q9ULQ0",
  "term_id": "GO:0035331"
}